{
  "gene_name": "Olfactory receptor 4K2",
  "gene": "UniProtKB:Q8NGD2",
  "gene_symbol": "OR4K2",
  "term_id": "UNKNOWN:0003",
  "term_label": "Unknown cellular component"
}